{
  "term_id": "UNKNOWN:0002",
  "gene_symbol": "OR8K5",
  "term_label": "Unknown biological process",
  "gene": "UniProtKB:Q8NH50",
  "gene_name": "Olfactory receptor 8K5"
}